{
  "term_label": "Unknown molecular function",
  "gene": "UniProtKB:A0A0J9YVP2",
  "gene_name": "Immunoglobulin heavy joining 6 (Fragment)",
  "gene_symbol": "IGHJ6",
  "term_id": "UNKNOWN:0001"
}